{
  "term_id": "GO:0006043",
  "gene": "UniProtKB:Q8TDQ7",
  "gene_symbol": "GNPDA2",
  "term_label": "glucosamine catabolic process",
  "gene_name": "Glucosamine-6-phosphate isomerase 2"
}